GPI-mannose ethanolamine phosphate phosphodiesterase activity [GO:0062050] (molecular function) References: PMID:19837036 Relationships: is a type of phosphoric diester hydrolase activity [GO:0008081] Definition: A phosphoric diester hydrolase activity that removes the ethanolamine phosphate from mannose 2 of a GPI anchor.